{
  "gene_symbol": "NEUROD1",
  "term_label": "sensory organ development",
  "gene_name": "Neurogenic differentiation factor 1",
  "gene": "UniProtKB:Q13562",
  "term_id": "GO:0007423"
}